{
  "term_label": "centrosome",
  "term_id": "GO:0005813",
  "gene": "UniProtKB:Q8N137",
  "gene_name": "Centrobin",
  "gene_symbol": "CNTROB"
}